{
  "gene": "UniProtKB:Q10589",
  "gene_name": "Bone marrow stromal antigen 2",
  "term_label": "cell surface",
  "gene_symbol": "BST2",
  "term_id": "GO:0009986"
}